vascular transport [GO:0010232] (biological process) Definition: The directed movement of substances, into, out of or within a cell, either in a vascular tissue or in the vascular membrane. Sources: GOC:sm Relationships: is a type of vascular process in circulatory system [GO:0003018]; is a type of transport [GO:0006810] Subtypes: phloem transport [GO:0010233], transport across blood-brain barrier [GO:0150104], transport across blood-cerebrospinal fluid barrier [GO:0150195]